aldose-1-phosphate adenylyltransferase activity [GO:0047346] (molecular function) Also known as: ADP-sugar phosphorylase activity, sugar-1-phosphate adenylyltransferase activity, ADP:aldose-1-phosphate adenylyltransferase activity, ADP sugar phosphorylase activity, ADP-aldose phosphorylase activity, ADP:alpha-D-aldose-1-phosphate adenylyltransferase activity, ADPaldose phosphorylase activity, adenosine diphosphate glucose:orthophosphate adenylyltransferase activity, adenosine diphosphosugar phosphorylase activity Sources: EC:2.7.7.36, MetaCyc:2.7.7.36-RXN Definition: Catalysis of the reaction: aldose 1-phosphate + ADP = phosphate + ADP-aldose. Relationships: is a type of adenylyltransferase activity [GO:0070566]